abscisic acid metabolic process [GO:0009687] (biological process) Also known as: abscisic acid metabolism Relationships: is a type of sesquiterpenoid metabolic process [GO:0006714]; is_a monocarboxylic acid metabolic process [GO:0032787]; is a type of olefinic compound metabolic process [GO:0120254]; is a type of tertiary alcohol metabolic process [GO:1902644] Definition: The chemical reactions and pathways involving abscisic acid, 5-(1-hydroxy-2,6,6,trimethyl-4-oxocyclohex-2-en-1-y1)-3-methylpenta-2,4-dienoic acid. Sources: ISBN:0387969845 Subtypes: abscisic acid biosynthetic process [GO:0009688], abscisic acid catabolic process [GO:0046345]